{
  "term_label": "calcium ion binding",
  "term_id": "GO:0005509",
  "gene_name": "Putative oncomodulin-2",
  "gene_symbol": "OCM2",
  "gene": "UniProtKB:P0CE71"
}